cell wall (1->3)-alpha-glucan biosynthetic process [GO:0070598] (biological process) Regulation: regulated by regulation of cell wall (1->3)-alpha-glucan biosynthetic process [GO:0070608] Definition: The chemical reactions and pathways resulting in the formation of (1->3)-alpha-D-glucans, compounds composed of glucose residues linked by (1->3)-alpha-glucosidic bonds, found in the walls of cells. Subtypes: fungal-type cell wall (1->3)-alpha-glucan biosynthetic process [GO:0070600] Sources: GOC:mah Also known as: cell wall 1,3-alpha-glucan anabolism, cell wall 1,3-alpha-glucan biosynthesis, cell wall 1,3-alpha-glucan biosynthetic process, cell wall 1,3-alpha-glucan formation, cell wall 1,3-alpha-glucan synthesis, cell wall alpha-1,3-glucan anabolism, cell wall alpha-1,3-glucan biosynthesis, cell wall alpha-1,3-glucan biosynthetic process, cell wall alpha-1,3-glucan formation, cell wall alpha-1,3-glucan synthesis Relationships: is a type of cell wall polysaccharide biosynthetic process [GO:0070592]; is a type of GO:0070596; is a type of cell wall (1->3)-alpha-glucan metabolic process [GO:0070597]